{
  "term_id": "GO:0009986",
  "gene_symbol": "ITGA2",
  "gene": "UniProtKB:P17301",
  "gene_name": "Integrin alpha-2",
  "term_label": "cell surface"
}